{
  "gene": "UniProtKB:Q969S3",
  "gene_symbol": "ZNF622",
  "gene_name": "Cytoplasmic 60S subunit biogenesis factor ZNF622",
  "term_label": "ribosomal large subunit biogenesis",
  "term_id": "GO:0042273"
}